{
  "term_id": "GO:0051965",
  "gene_symbol": "AMIGO3",
  "term_label": "positive regulation of synapse assembly",
  "gene": "UniProtKB:Q86WK7",
  "gene_name": "Amphoterin-induced protein 3"
}